{
  "term_id": "GO:0072659",
  "gene_symbol": "PALS1",
  "gene_name": "Protein PALS1",
  "term_label": "protein localization to plasma membrane",
  "gene": "UniProtKB:Q8N3R9"
}